{
  "term_label": "trans-2-enoyl-CoA reductase (NADPH) activity",
  "gene_symbol": "PECR",
  "gene": "UniProtKB:Q9BY49",
  "gene_name": "Peroxisomal trans-2-enoyl-CoA reductase",
  "term_id": "GO:0019166"
}